{
  "gene": "UniProtKB:P0DUD3",
  "gene_symbol": "SPDYE14",
  "term_label": "protein kinase binding",
  "term_id": "GO:0019901",
  "gene_name": "Putative speedy protein E14"
}